negative regulation of nucleoside metabolic process [GO:0045978] (biological process) Sources: GOC:go_curators Definition: Any process that stops, prevents, or reduces the frequency, rate or extent of the chemical reactions and pathways involving nucleosides. Also known as: down regulation of nucleoside metabolic process, down-regulation of nucleoside metabolic process, downregulation of nucleoside metabolic process, negative regulation of nucleoside metabolism, inhibition of nucleoside metabolic process Relationships: is a type of regulation of nucleoside metabolic process [GO:0009118]; is a type of negative regulation of nucleobase-containing compound metabolic process [GO:0045934]; is a type of negative regulation of small molecule metabolic process [GO:0062014]; negatively regulates nucleoside metabolic process [GO:0009116]